{
  "gene": "UniProtKB:Q8NDZ4",
  "term_label": "cardiac muscle cell proliferation",
  "term_id": "GO:0060038",
  "gene_symbol": "DIPK2A",
  "gene_name": "Divergent protein kinase domain 2A"
}